regulation of retinal cell programmed cell death [GO:0046668] (biological process) Subtypes: GO:0046669, positive regulation of retinal cell programmed cell death [GO:0046670], GO:0046671 Sources: GOC:ai, GOC:tb Also known as: regulation of retinal programmed cell death Relationships: is_a regulation of programmed cell death [GO:0043067]; is a type of GO:0050793; regulates GO:0046666 Definition: Any process that modulates the frequency, rate or extent of programmed cell death that occurs in the retina.